3-butenylglucosinolate 2-hydroxylase activity [GO:0062131] (molecular function) Definition: Catalysis of the reaction: gluconapin + a reduced electron acceptor + O2 = xi-progoitrin + an oxidized electron acceptor + H2O. References: PMID:18945935 Also known as: But-3-enyl Glucosinolate-2-hydroxylase activity Relationships: is a type of dioxygenase activity [GO:0051213]